{
  "gene_symbol": "SLC13A2",
  "gene_name": "Solute carrier family 13 member 2",
  "gene": "UniProtKB:Q13183",
  "term_label": "sodium:dicarboxylate symporter activity",
  "term_id": "GO:0017153"
}